{
  "gene": "UniProtKB:Q13418",
  "term_id": "GO:0005102",
  "term_label": "signaling receptor binding",
  "gene_name": "Integrin-linked protein kinase",
  "gene_symbol": "ILK"
}